{
  "term_label": "nucleus",
  "term_id": "GO:0005634",
  "gene_symbol": "TRAPPC2L",
  "gene": "UniProtKB:Q9UL33",
  "gene_name": "Trafficking protein particle complex subunit 2-like protein"
}